apigenin 4'-O-methyltransferase activity [GO:0030754] (molecular function) Definition: Catalysis of the reaction: S-adenosyl-L-methionine + 5,7,4'-trihydroxyflavone = S-adenosyl-L-homocysteine + 4'-methoxy-5,7-dihydroxyflavone. Relationships: is a type of S-adenosylmethionine-dependent methyltransferase activity [GO:0008757] Also known as: flavonoid O-methyltransferase activity, S-adenosyl-L-methionine:5,7,4'-trihydroxyflavone 4'-O-methyltransferase activity, flavonoid methyltransferase activity Sources: EC:2.1.1.75